{
  "gene_name": "Semaphorin-3C",
  "term_label": "neural crest cell migration",
  "gene_symbol": "SEMA3C",
  "gene": "UniProtKB:Q99985",
  "term_id": "GO:0001755"
}